{
  "term_label": "axon guidance",
  "gene_symbol": "EPHA4",
  "gene_name": "Ephrin type-A receptor 4",
  "term_id": "GO:0007411",
  "gene": "UniProtKB:P54764"
}